{
  "gene_name": "PH and SEC7 domain-containing protein 4",
  "gene_symbol": "PSD4",
  "gene": "UniProtKB:Q8NDX1",
  "term_label": "ruffle membrane",
  "term_id": "GO:0032587"
}